chromium ion transmembrane transporter activity [GO:0070835] (molecular function) Definition: Enables the transfer of chromium (Cr) ions from one side of a membrane to the other. Sources: GOC:mah, GOC:yaf Relationships: is a type of transmembrane transporter activity [GO:0022857]